negative regulation of response to food [GO:0032096] (biological process) Sources: GOC:add Also known as: down regulation of response to food, down-regulation of response to food, downregulation of response to food, inhibition of response to food Subtypes: GO:0032099, GO:2000140 Relationships: is a type of regulation of response to food [GO:0032095]; is a type of GO:0032108; negatively regulates response to food [GO:0032094] Definition: Any process that stops, prevents, or reduces the frequency, rate or extent of a response to a food stimulus.